{
  "term_id": "GO:0031175",
  "gene_symbol": "GDNF",
  "term_label": "neuron projection development",
  "gene": "UniProtKB:P39905",
  "gene_name": "Glial cell line-derived neurotrophic factor"
}